regulation of floral organ abscission [GO:0060860] (biological process) Relationships: is a type of regulation of developmental process [GO:0050793]; is a type of GO:2000241; RO_0002211 floral organ abscission [GO:0010227] Subtypes: positive regulation of floral organ abscission [GO:0060861], negative regulation of floral organ abscission [GO:0060862], GO:0060863 Definition: Any process that modulates the rate, frequency, or extent of floral organ abscission, the controlled shedding of floral organs. Sources: GOC:dph, GOC:sdb_2009, GOC:tb